{
  "gene_name": "E3 ubiquitin-protein ligase TRIM58",
  "term_label": "innate immune response",
  "gene": "UniProtKB:Q8NG06",
  "term_id": "GO:0045087",
  "gene_symbol": "TRIM58"
}